{
  "gene": "UniProtKB:Q9WJR5",
  "gene_symbol": "ERVK-19",
  "term_label": "Unknown cellular component",
  "gene_name": "Endogenous retrovirus group K member 19 Pol protein",
  "term_id": "UNKNOWN:0003"
}